{
  "gene_name": "Histone H2B type 1-O",
  "gene": "UniProtKB:P23527",
  "term_label": "innate immune response in mucosa",
  "term_id": "GO:0002227",
  "gene_symbol": "H2BC17"
}